{
  "gene": "UniProtKB:A6NIU2",
  "term_id": "UNKNOWN:0003",
  "gene_symbol": "LINC01549",
  "term_label": "Unknown cellular component",
  "gene_name": "Putative uncharacterized protein encoded by LINC01549"
}